{
  "term_id": "UNKNOWN:0002",
  "term_label": "Unknown biological process",
  "gene_name": "S100P-binding protein",
  "gene": "UniProtKB:Q96BU1",
  "gene_symbol": "S100PBP"
}